{
  "term_id": "GO:0031116",
  "term_label": "positive regulation of microtubule polymerization",
  "gene_name": "CAP-Gly domain-containing linker protein 1",
  "gene": "UniProtKB:P30622",
  "gene_symbol": "CLIP1"
}